mitotic DNA replication [GO:1902969] (biological process) Relationships: is a type of nuclear DNA replication [GO:0033260]; is a type of mitotic cell cycle process [GO:1903047] Regulation: regulated by regulation of mitotic cell cycle DNA replication [GO:1903463]; RO_0002212 by negative regulation of mitotic cell cycle DNA replication [GO:1903464]; positively regulated by GO:1903465 Sources: GOC:TermGenie, GO_REF:0000060 Subtypes: mitotic DNA-templated DNA replication [GO:1990506] Also known as: DNA replication involved in S phase involved in mitotic cell cycle, DNA replication involved in S-phase involved in mitotic cell cycle, mitotic cell cycle DNA replication, mitotic nuclear cell cycle DNA replication, DNA replication during S phase involved in mitotic cell cycle, nuclear cell cycle DNA replication involved in mitotic cell cycle Definition: Any nuclear DNA replication that is involved in a mitotic cell cycle.